{
  "gene_symbol": "TCTN3",
  "gene_name": "Tectonic-3",
  "term_id": "UNKNOWN:0003",
  "term_label": "Unknown cellular component",
  "gene": "UniProtKB:Q6NUS6"
}